{
  "gene_name": "Regulator of microtubule dynamics protein 3",
  "gene": "UniProtKB:Q96TC7",
  "term_id": "GO:0005876",
  "gene_symbol": "RMDN3",
  "term_label": "spindle microtubule"
}